{
  "gene_symbol": "TEX11",
  "term_label": "synaptonemal complex assembly",
  "gene": "UniProtKB:Q8IYF3",
  "gene_name": "Testis-expressed protein 11",
  "term_id": "GO:0007130"
}